{
  "term_label": "Unknown molecular function",
  "gene_symbol": "MTFR1",
  "gene": "UniProtKB:Q15390",
  "gene_name": "Mitochondrial fission regulator 1",
  "term_id": "UNKNOWN:0001"
}